entry into reproductive diapause [GO:0055116] (biological process) Definition: The dormancy process that results in entry into reproductive diapause. Reproductive diapause is a form of diapause where the organism itself will remain fully active, including feeding and other routine activities, but the reproductive organs experience a tissue-specific reduction in metabolism, with characteristic triggering and releasing stimuli. Regulation: regulated by regulation of entry into reproductive diapause [GO:0061963]; negatively regulated by GO:0061964; positively regulated by positive regulation of entry into reproductive diapause [GO:0061965] Sources: GOC:ds, GOC:jid, GOC:mah Relationships: is a type of GO:0055115